plasma membrane acetate transport [GO:0006847] (biological process) Relationships: is a type of acetate transmembrane transport [GO:0035433] Sources: GOC:ai Definition: The directed movement of acetate across a plasma membrane.